{
  "gene_name": "Acyl-CoA 6-desaturase",
  "gene": "UniProtKB:O95864",
  "gene_symbol": "FADS2",
  "term_label": "lipid metabolic process",
  "term_id": "GO:0006629"
}